regulation of interferon-beta production [GO:0032648] (biological process) Also known as: regulation of IFN-beta production, regulation of interferon-beta biosynthetic process, regulation of interferon-beta secretion Relationships: is a type of GO:0032479; regulates GO:0032608 References: PMID:15546383 Sources: GOC:mah Definition: Any process that modulates the frequency, rate, or extent of interferon-beta production. Subtypes: negative regulation of interferon-beta production [GO:0032688], positive regulation of interferon-beta production [GO:0032728]